invasive growth in response to glucose limitation [GO:0001403] (biological process) Definition: A growth pattern exhibited by budding haploid cells under certain growth conditions, in which cells retain the typical axial budding pattern of haploids, but become elongated and fail to separate after division; during growth on a solid substrate, this results in penetration of cells into the agar medium. An example of this process is found in Saccharomyces cerevisiae. Relationships: is a type of GO:0036267 Note: Note that this term should not be used to describe the invasion of host tissues by pathogenic organisms, which is described by the biological process term 'entry into host ; GO:0044409', nor should it be used to describe growth of diseased cells of an organism into the surrounding normal tissue, which is outside of the scope of GO. Regulation: regulated by regulation of invasive growth in response to glucose limitation [GO:2000217]; RO_0002212 by negative regulation of invasive growth in response to glucose limitation [GO:2000218]; positively regulated by positive regulation of invasive growth in response to glucose limitation [GO:2000219] Also known as: colony morphology References: PMID:9728395 Sources: GOC:mcc